4-aminobutyrate:pyruvate transaminase activity [GO:0034387] (molecular function) Sources: EC:2.6.1.96 Also known as: gamma-aminobutyric acid pyruvate transaminase activity Relationships: is a type of GO:0008483 Definition: Catalysis of the reaction: 4-aminobutanoate + pyruvate = succinate semialdehyde + alanine. Also converts glyoxylate to glycine.